{
  "gene_name": "Chromobox protein homolog 8",
  "term_label": "chromatin",
  "gene": "UniProtKB:Q9HC52",
  "gene_symbol": "CBX8",
  "term_id": "GO:0000785"
}